{
  "term_label": "positive regulation of vascular endothelial growth factor production",
  "gene_symbol": "SULF1",
  "term_id": "GO:0010575",
  "gene": "UniProtKB:Q8IWU6",
  "gene_name": "Extracellular sulfatase Sulf-1"
}